{
  "term_label": "cytosol",
  "gene_name": "Fructose-1,6-bisphosphatase isozyme 2",
  "gene_symbol": "FBP2",
  "gene": "UniProtKB:O00757",
  "term_id": "GO:0005829"
}